{
  "gene": "UniProtKB:O43897",
  "term_id": "GO:0009953",
  "term_label": "dorsal/ventral pattern formation",
  "gene_symbol": "TLL1",
  "gene_name": "Tolloid-like protein 1"
}